{
  "gene": "UniProtKB:P17544",
  "gene_symbol": "ATF7",
  "term_label": "cAMP response element binding",
  "term_id": "GO:0035497",
  "gene_name": "Cyclic AMP-dependent transcription factor ATF-7"
}